regulation of purine nucleotide biosynthetic process [GO:1900371] (biological process) Definition: Any process that modulates the frequency, rate or extent of purine nucleotide biosynthetic processes. Subtypes: negative regulation of purine nucleotide biosynthetic process [GO:1900372], GO:1900373, regulation of 'de novo' NAD biosynthetic process from L-tryptophan [GO:1905012], GO:2001169 Relationships: is a type of regulation of nucleotide biosynthetic process [GO:0030808]; is a type of regulation of purine nucleotide metabolic process [GO:1900542]; RO_0002211 GO:0006164 Sources: GOC:TermGenie, GOC:go_curators Also known as: regulation of purine nucleotide anabolism, regulation of purine nucleotide biosynthesis, regulation of purine nucleotide formation, regulation of purine nucleotide synthesis